{
  "gene_symbol": "SLC25A30",
  "term_label": "Unknown biological process",
  "term_id": "UNKNOWN:0002",
  "gene_name": "Kidney mitochondrial carrier protein 1",
  "gene": "UniProtKB:Q5SVS4"
}